{
  "term_id": "GO:0031053",
  "term_label": "primary miRNA processing",
  "gene_name": "Ribonuclease 3",
  "gene": "UniProtKB:Q9NRR4",
  "gene_symbol": "DROSHA"
}